{
  "term_label": "postsynaptic density membrane",
  "gene_name": "Plasma membrane calcium-transporting ATPase 2",
  "gene": "UniProtKB:Q01814",
  "gene_symbol": "ATP2B2",
  "term_id": "GO:0098839"
}